{
  "gene": "UniProtKB:Q9NQT6",
  "gene_name": "Fascin-3",
  "term_id": "GO:0005737",
  "term_label": "cytoplasm",
  "gene_symbol": "FSCN3"
}